{
  "gene_name": "Proton channel OTOP2",
  "gene_symbol": "OTOP2",
  "term_id": "GO:0015252",
  "term_label": "proton channel activity",
  "gene": "UniProtKB:Q7RTS6"
}